histone H3K4 dimethyltransferase activity [GO:0140946] (molecular function) Relationships: is a type of histone H3K4 methyltransferase activity [GO:0042800] Sources: RHEA:64448 Also known as: histone H3-K4 dimethylation, histone H3K4 dimethylation, histone H3K4 dimethylase activity, histone lysine N-dimethyltransferase activity (H3-K4 specific) Definition: Catalysis of the reaction: L-lysyl4-[histone H3] + 2 S-adenosyl-L-methionine = 2 H+ + N6,N6-dimethyl-L-lysyl4-[histone H3] + 2 S-adenosyl-L-homocysteine. This reaction is the successive addition of two methyl groups to the unmethylated lysine residue at position 4 of histone H3, producing histone H3K4me2. Note: Comment: Note that the residue position corresponds to the canonical human H3 histone (UniProtKB:P84243); this residue is conserved across all eukaryotes. Residue 1 is the first residue following removal of the initiating Methionine (Met). Note that each histone is encoded by multiple genes, and sequences may vary across different genes within an organism.